{
  "term_id": "GO:0045672",
  "gene_symbol": "UNQ5830/PRO19650/PRO19816",
  "gene": "UniProtKB:Q6UY13",
  "term_label": "positive regulation of osteoclast differentiation",
  "gene_name": "Putative uncharacterized protein UNQ5830_PRO19650_PRO19816"
}